{
  "gene_name": "Nuclear factor erythroid 2-related factor 3",
  "gene_symbol": "NFE2L3",
  "gene": "UniProtKB:Q9Y4A8",
  "term_label": "regulation of transcription by RNA polymerase II",
  "term_id": "GO:0006357"
}